{
  "term_label": "Unknown biological process",
  "gene": "UniProtKB:O76021",
  "term_id": "UNKNOWN:0002",
  "gene_name": "Ribosomal L1 domain-containing protein 1",
  "gene_symbol": "RSL1D1"
}